{
  "gene": "UniProtKB:P10599",
  "term_label": "Unknown molecular function",
  "term_id": "UNKNOWN:0001",
  "gene_symbol": "TXN",
  "gene_name": "Thioredoxin"
}